{
  "gene_name": "Protein odd-skipped-related 1",
  "term_id": "GO:0005634",
  "term_label": "nucleus",
  "gene": "UniProtKB:Q8TAX0",
  "gene_symbol": "OSR1"
}